{
  "term_id": "GO:0005737",
  "gene_name": "Ankyrin repeat domain-containing protein 54",
  "gene_symbol": "ANKRD54",
  "gene": "UniProtKB:Q6NXT1",
  "term_label": "cytoplasm"
}